laminaribiose binding [GO:0044588] (molecular function) Definition: Binding to laminaribiose, a disaccharide. Relationships: is a type of oligosaccharide binding [GO:0070492] Sources: GOC:mengo_curators, GOC:tt